{
  "term_id": "GO:0090307",
  "gene": "UniProtKB:O43670",
  "gene_name": "BUB3-interacting and GLEBS motif-containing protein ZNF207",
  "term_label": "mitotic spindle assembly",
  "gene_symbol": "ZNF207"
}